carbohydrate:monoatomic cation symporter activity [GO:0005402] (molecular function) Relationships: is a type of GO:0015144; is a type of solute:monoatomic cation symporter activity [GO:0015294] Subtypes: GO:0005351, GO:0005412, GO:0008520, sucrose:monoatomic cation symporter activity [GO:0009669], galactose:sodium symporter activity [GO:0015371], glycoside-pentoside-hexuronide:cation symporter activity [GO:0015486], GO:0015487, mannose:sodium symporter activity [GO:0140929], fructose:sodium symporter activity [GO:0140930] Definition: Enables the transfer of a solute or solutes from one side of a membrane to the other according to the reaction: sugar(out) + cation(out) = sugar(in) + cation(in). Also known as: carbohydrate:cation symporter activity, cation/sugar symporter activity, cation:sugar symporter activity, sugar:cation symporter activity Sources: GOC:ai